positive regulation of sphingolipid mediated signaling pathway [GO:1902070] (biological process) References: PMID:20870412 Sources: GOC:TermGenie Relationships: is a type of GO:0009967; is a type of regulation of sphingolipid mediated signaling pathway [GO:1902068]; positively regulates sphingolipid mediated signaling pathway [GO:0090520] Definition: Any process that activates or increases the frequency, rate or extent of sphingolipid signaling. Also known as: up regulation of sphingolipid mediated signaling pathway, up-regulation of sphingolipid mediated signaling pathway, upregulation of sphingolipid mediated signaling pathway, activation of sphingolipid mediated signaling pathway, activation of sphingolipid signaling pathway, positive regulation of sphingolipid signaling pathway, up regulation of sphingolipid signaling pathway, up-regulation of sphingolipid signaling pathway, upregulation of sphingolipid signaling pathway